{
  "gene_symbol": "CLDN9",
  "gene": "UniProtKB:O95484",
  "gene_name": "Claudin-9",
  "term_label": "virus receptor activity",
  "term_id": "GO:0001618"
}